{
  "gene_name": "E3 ubiquitin-protein ligase RNF6",
  "gene": "UniProtKB:Q9Y252",
  "term_label": "protein ubiquitination",
  "gene_symbol": "RNF6",
  "term_id": "GO:0016567"
}